positive regulation of fumigaclavine C biosynthetic process [GO:1900839] (BP) Also known as: up regulation of fumigaclavine C biosynthetic process, up-regulation of fumigaclavine C biosynthetic process, upregulation of fumigaclavine C biosynthetic process Relationships: is a type of GO:1900824; is a type of GO:1900837; positively regulates GO:1900809 Sources: GOC:TermGenie, GOC:di Definition: Any process that activates or increases the frequency, rate or extent of fumigaclavine C biosynthetic process.